negative regulation of blood coagulation [GO:0030195] (biological process) Definition: Any process that stops, prevents, or reduces the frequency, rate or extent of blood coagulation. Subtypes: negative regulation of platelet activation [GO:0010544], fibrinolysis [GO:0042730], positive regulation of fibrinolysis [GO:0051919], negative regulation of blood coagulation, common pathway [GO:2000261], negative regulation of blood coagulation, extrinsic pathway [GO:2000264], GO:2000267 Sources: GOC:mah Also known as: down regulation of blood coagulation, down-regulation of blood coagulation, downregulation of blood coagulation, inhibition of blood coagulation Relationships: is a type of GO:0030193; is_a negative regulation of coagulation [GO:0050819]; is a type of negative regulation of wound healing [GO:0061045]; is a type of negative regulation of hemostasis [GO:1900047]; negatively regulates blood coagulation [GO:0007596]